regulation of monocyte chemotaxis [GO:0090025] (biological process) Definition: Any process that modulates the frequency, rate, or extent of monocyte chemotaxis. Sources: GOC:dph, GOC:tb Relationships: is a type of regulation of leukocyte chemotaxis [GO:0002688]; is a type of GO:0071675; RO_0002211 monocyte chemotaxis [GO:0002548] Subtypes: positive regulation of monocyte chemotaxis [GO:0090026], negative regulation of monocyte chemotaxis [GO:0090027]